regulation of quinolinate biosynthetic process [GO:1904984] (biological process) References: PMID:12140278, PMID:19843166 Sources: GOC:PARL, GOC:TermGenie, GOC:bf, GO_REF:0000058 Definition: Any process that modulates the frequency, rate or extent of quinolinate biosynthetic process. Subtypes: negative regulation of quinolinate biosynthetic process [GO:1904985], positive regulation of quinolinate biosynthetic process [GO:1904986] Also known as: regulation of quinolinate anabolism, regulation of quinolinate biosynthesis, regulation of quinolinate formation, regulation of quinolinate synthesis Relationships: is a type of regulation of biosynthetic process [GO:0009889]; is a type of GO:0062012; regulates quinolinate biosynthetic process [GO:0019805]